{
  "gene_name": "Putative POU domain, class 5, transcription factor 1B",
  "gene_symbol": "POU5F1B",
  "term_id": "GO:0006357",
  "gene": "UniProtKB:Q06416",
  "term_label": "regulation of transcription by RNA polymerase II"
}